{
  "gene_symbol": "CXCL8",
  "term_label": "cellular response to lipopolysaccharide",
  "term_id": "GO:0071222",
  "gene": "UniProtKB:P10145",
  "gene_name": "Interleukin-8"
}